{
  "gene": "UniProtKB:Q9BQQ7",
  "gene_name": "Receptor-transporting protein 3",
  "term_id": "GO:0051205",
  "term_label": "protein insertion into membrane",
  "gene_symbol": "RTP3"
}